{
  "gene_name": "GMP synthase [glutamine-hydrolyzing]",
  "term_label": "cytosol",
  "term_id": "GO:0005829",
  "gene_symbol": "GMPS",
  "gene": "UniProtKB:P49915"
}